intermediate mesodermal cell fate determination [GO:0048394] (biological process) Sources: GOC:dgh Definition: The process in which a cell becomes capable of differentiating autonomously into a intermediate mesoderm cell regardless of its environment; upon determination, the cell fate cannot be reversed. Also known as: intermediate mesoderm cell fate determination Regulation: regulated by GO:0048395; negatively regulated by negative regulation of intermediate mesodermal cell fate determination [GO:0048396]; positively regulated by positive regulation of intermediate mesodermal cell fate determination [GO:0048397] Relationships: is a type of mesodermal cell fate determination [GO:0007500]; is part of intermediate mesodermal cell fate commitment [GO:0048393]